{
  "gene": "UniProtKB:P10276",
  "term_label": "negative regulation of transcription by RNA polymerase II",
  "gene_name": "Retinoic acid receptor alpha",
  "term_id": "GO:0000122",
  "gene_symbol": "RARA"
}